{
  "term_id": "UNKNOWN:0001",
  "gene_name": "Low-density lipoprotein receptor class A domain-containing protein 3",
  "gene_symbol": "LDLRAD3",
  "gene": "UniProtKB:Q86YD5",
  "term_label": "Unknown molecular function"
}